{
  "term_label": "cytoplasm",
  "term_id": "GO:0005737",
  "gene": "UniProtKB:Q13117",
  "gene_name": "Deleted in azoospermia protein 2",
  "gene_symbol": "DAZ2"
}